axial mesodermal cell fate determination [GO:0048323] (biological process) Also known as: axial mesoderm cell fate determination Relationships: is a type of GO:0007500; is part of axial mesodermal cell fate commitment [GO:0048322] Definition: The process in which a cell becomes capable of differentiating autonomously into an axial mesoderm cell regardless of its environment; upon determination, the cell fate cannot be reversed. Regulation: regulated by regulation of axial mesodermal cell fate determination [GO:0048324]; negatively regulated by negative regulation of axial mesodermal cell fate determination [GO:0048325]; positively regulated by positive regulation of axial mesodermal cell fate determination [GO:0048326] Sources: GOC:dgh